kaempferide 3-O-methyltransferase activity [GO:0102451] (molecular function) Definition: Catalysis of the reaction: kaempferide + S-adenosyl-L-methionine = 3,4'-O-dimethylkaempferol + H+ + S-adenosyl-L-homocysteine. Sources: RHEA:74755 Relationships: is a type of methyltransferase activity [GO:0008168]